{
  "gene": "UniProtKB:P30154",
  "term_id": "GO:0051225",
  "gene_symbol": "PPP2R1B",
  "gene_name": "Serine_threonine-protein phosphatase 2A 65 kDa regulatory subunit A beta isoform",
  "term_label": "spindle assembly"
}